{
  "gene_symbol": "TTBK2",
  "gene": "UniProtKB:Q6IQ55",
  "gene_name": "Tau-tubulin kinase 2",
  "term_id": "GO:0035869",
  "term_label": "ciliary transition zone"
}